{
  "gene_symbol": "BOC",
  "term_id": "GO:0007411",
  "gene": "UniProtKB:Q9BWV1",
  "gene_name": "Brother of CDO",
  "term_label": "axon guidance"
}